axonemal central pair [GO:0097540] (cellular component) Also known as: central pair, axonemal microtubule central pair, axoneme central pair, axoneme microtubule central pair, central-pair microtubules Definition: Part of the axoneme consisting of the inner two microtubule doublets of the 9+2 axoneme occurring in most motile cilia. References: PMID:24283352 Sources: GOC:cilia, GOC:krc Relationships: is_a GO:0110165; is part of axonemal central apparatus [GO:1990716]; has part C1 axonemal microtubule [GO:1990719]; has part GO:1990720